kinociliary basal body [GO:1902636] (cellular component) Relationships: is a type of ciliary basal body [GO:0036064]; is part of kinocilium [GO:0060091] References: PMID:15855039, PMID:15882574 Sources: GOC:TermGenie, GOC:cilia, GOC:krc, GO_REF:0000064 Also known as: cilial basal body of kinocilium, ciliary basal body of kinocilium, cilium basal body of kinocilium, kinocilial basal body, kinocilium basal body, kinocilium ciliary basal body, microtubule basal body of kinocilium Definition: A ciliary basal body that is part of a kinocilium.